versicolorin reductase activity [GO:0042469] (MF) Definition: Catalysis of the reduction of versicolorin A to sterigmatocystin. References: PMID:1339261 Relationships: is a type of oxidoreductase activity, acting on CH-OH group of donors [GO:0016614]